{
  "gene": "UniProtKB:H3BV60",
  "gene_name": "Transforming growth factor-beta receptor type 3-like protein",
  "term_label": "cell migration",
  "term_id": "GO:0016477",
  "gene_symbol": "TGFBR3L"
}